{
  "gene": "UniProtKB:Q9BUZ4",
  "term_label": "cytoplasm",
  "term_id": "GO:0005737",
  "gene_name": "TNF receptor-associated factor 4",
  "gene_symbol": "TRAF4"
}